positive regulation of plasminogen activation [GO:0010756] (biological process) Sources: GOC:BHF, GOC:dph, GOC:tb Definition: Any process that increases the rate, frequency or extent of plasminogen activation. Plasminogen activation is the process in which plasminogen is processed to plasmin. Relationships: is_a GO:0010755; is a type of positive regulation of protein processing [GO:0010954]; positively regulates plasminogen activation [GO:0031639]